{
  "gene_symbol": "FUT6",
  "gene": "UniProtKB:P51993",
  "gene_name": "4-galactosyl-N-acetylglucosaminide 3-alpha-L-fucosyltransferase FUT6",
  "term_id": "GO:0005794",
  "term_label": "Golgi apparatus"
}